deoxynucleotide transport [GO:0030302] (biological process) Relationships: is a type of nucleotide transport [GO:0006862]; is a type of carbohydrate derivative transport [GO:1901264] Definition: The directed movement of a deoxynucleotide, a deoxyribonucleoside in ester linkage to phosphate, commonly at the 5' position of deoxyribose, into, out of or within a cell. Sources: GOC:mah, ISBN:0198506732